{
  "term_label": "receptor-mediated endocytosis",
  "term_id": "GO:0006898",
  "gene_symbol": "LY75",
  "gene_name": "Lymphocyte antigen 75",
  "gene": "UniProtKB:O60449"
}